{
  "gene_name": "Tropomodulin-2",
  "term_label": "actin filament organization",
  "term_id": "GO:0007015",
  "gene": "UniProtKB:Q9NZR1",
  "gene_symbol": "TMOD2"
}